{
  "term_label": "Unknown cellular component",
  "gene_symbol": "CRYGD",
  "gene_name": "Gamma-crystallin D",
  "term_id": "UNKNOWN:0003",
  "gene": "UniProtKB:P07320"
}